{
  "gene": "UniProtKB:P17036",
  "term_id": "GO:0006357",
  "gene_symbol": "ZNF3",
  "term_label": "regulation of transcription by RNA polymerase II",
  "gene_name": "Zinc finger protein 3"
}